regulation of apoptotic process [GO:0042981] (biological process) Definition: Any process that modulates the occurrence or rate of cell death by apoptotic process. Also known as: regulation of apoptosis, apoptosis regulator activity Note: This term should only be used when it is not possible to determine which phase or subtype of the apoptotic process is regulated by a gene product. Whenever detailed information is available, the more granular children terms should be used. Subtypes: GO:0010660, regulation of myeloid cell apoptotic process [GO:0033032], regulation of glial cell apoptotic process [GO:0034350], GO:0043065, negative regulation of apoptotic process [GO:0043066], regulation of neuron apoptotic process [GO:0043523], GO:0060785, regulation of apoptotic process in bone marrow cell [GO:0071865], GO:1901692, regulation of epithelial cell apoptotic process [GO:1904035], GO:1904520, regulation of fat cell apoptotic process [GO:1904649], regulation of apoptotic process involved in development [GO:1904748], regulation of leukocyte apoptotic process [GO:2000106], regulation of anoikis [GO:2000209], regulation of fibroblast apoptotic process [GO:2000269], regulation of endothelial cell apoptotic process [GO:2000351], regulation of mesenchymal cell apoptotic process [GO:2001053], regulation of apoptotic signaling pathway [GO:2001233] Sources: GOC:jl, GOC:mtg_apoptosis Relationships: is_a regulation of programmed cell death [GO:0043067]; regulates apoptotic process [GO:0006915]